{
  "term_label": "keratin filament",
  "gene_symbol": "KRT72",
  "gene": "UniProtKB:Q14CN4",
  "gene_name": "Keratin, type II cytoskeletal 72",
  "term_id": "GO:0045095"
}